{
  "term_id": "UNKNOWN:0003",
  "gene": "UniProtKB:Q9NZ20",
  "term_label": "Unknown cellular component",
  "gene_symbol": "PLA2G3",
  "gene_name": "Group 3 secretory phospholipase A2"
}